{
  "gene_symbol": "COPB2",
  "gene": "UniProtKB:P35606",
  "gene_name": "Coatomer subunit beta'",
  "term_label": "endoplasmic reticulum to Golgi vesicle-mediated transport",
  "term_id": "GO:0006888"
}